{
  "gene_name": "Protein MTSS 2",
  "gene_symbol": "MTSS2",
  "gene": "UniProtKB:Q765P7",
  "term_id": "GO:0030031",
  "term_label": "cell projection assembly"
}